{
  "term_id": "GO:0005737",
  "gene_symbol": "RSPRY1",
  "gene": "UniProtKB:Q96DX4",
  "gene_name": "RING finger and SPRY domain-containing protein 1",
  "term_label": "cytoplasm"
}